{
  "term_id": "GO:0005634",
  "gene": "UniProtKB:P50461",
  "term_label": "nucleus",
  "gene_name": "Cysteine and glycine-rich protein 3",
  "gene_symbol": "CSRP3"
}